syringal lignin biosynthetic process [GO:1901066] (biological process) Definition: The chemical reactions and pathways resulting in the formation of syringal lignin. Sources: GOC:TermGenie, GOC:mengo_curators Also known as: S-lignin biosynthetic process, syringal lignin anabolism, syringal lignin biosynthesis, syringal lignin formation, syringal lignin synthesis Relationships: is a type of GO:0009809 Regulation: regulated by regulation of syringal lignin biosynthetic process [GO:1901428]; negatively regulated by negative regulation of syringal lignin biosynthetic process [GO:1901429]; positively regulated by positive regulation of syringal lignin biosynthetic process [GO:1901430]